{
  "gene_symbol": "EZHIP",
  "term_label": "Unknown biological process",
  "term_id": "UNKNOWN:0002",
  "gene_name": "EZH inhibitory protein",
  "gene": "UniProtKB:Q86X51"
}